{
  "gene_name": "Platelet glycoprotein IX",
  "gene": "UniProtKB:P14770",
  "term_label": "Unknown cellular component",
  "term_id": "UNKNOWN:0003",
  "gene_symbol": "GP9"
}